{
  "term_id": "UNKNOWN:0001",
  "gene_symbol": "LAMTOR2",
  "gene": "UniProtKB:Q9Y2Q5",
  "term_label": "Unknown molecular function",
  "gene_name": "Ragulator complex protein LAMTOR2"
}